proteasome binding [GO:0070628] (molecular function) Sources: GOC:mah Relationships: is a type of GO:0044877 Definition: Binding to a proteasome, a large multisubunit protein complex that catalyzes protein degradation.